{
  "term_id": "GO:0032467",
  "gene_symbol": "CDC14C",
  "term_label": "positive regulation of cytokinesis",
  "gene": "UniProtKB:A4D256",
  "gene_name": "Dual specificity protein phosphatase CDC14C"
}